{
  "gene_name": "Ataxin-2",
  "gene": "UniProtKB:Q99700",
  "gene_symbol": "ATXN2",
  "term_label": "cytoplasmic stress granule",
  "term_id": "GO:0010494"
}